diterpene phytoalexin biosynthetic process [GO:0051502] (biological process) Definition: The chemical reactions and pathways resulting in the formation of diterpene phytoalexins, terpenoids with 20 carbons produced by plants in response to environmental stresses. Relationships: is a type of GO:0016102; is a type of phytoalexin biosynthetic process [GO:0052315] Also known as: diterpene phytoalexin anabolism, diterpene phytoalexin biosynthesis, diterpene phytoalexin formation, diterpene phytoalexin synthesis Sources: GOC:ai